response to cell cycle checkpoint signaling [GO:0072396] (biological process) Definition: A process that occurs in response to signals generated as a result of cell cycle checkpoint signaling. Relationships: is a type of cellular response to biotic stimulus [GO:0071216]; is a type of cellular response to endogenous stimulus [GO:0071495] Regulation: regulated by regulation of response to cell cycle checkpoint signaling [GO:1902145]; positively regulated by positive regulation of response to cell cycle checkpoint signaling [GO:1902146] Sources: GOC:mtg_cell_cycle Also known as: cell cycle checkpoint effector process, response to signal involved in cell cycle checkpoint, G1/S transition checkpoint effector process, G2/M transition checkpoint effector process, response to G1/S transition checkpoint signaling, response to G2/M transition checkpoint signaling, response to signal involved in G1/S transition checkpoint, response to signal involved in G2/M transition checkpoint Subtypes: response to cytokinesis checkpoint signaling [GO:0072399], response to DNA integrity checkpoint signaling [GO:0072402], response to meiotic cell cycle checkpoint signaling [GO:0072410], response to mitotic cell cycle checkpoint signaling [GO:0072414], response to spindle checkpoint signaling [GO:0072417]